{
  "gene": "UniProtKB:Q8NCV1",
  "term_id": "GO:0006382",
  "gene_name": "Adenosine deaminase domain-containing protein 2",
  "gene_symbol": "ADAD2",
  "term_label": "adenosine to inosine editing"
}